{
  "gene_name": "von Willebrand factor A domain-containing protein 5B1",
  "term_label": "Unknown biological process",
  "term_id": "UNKNOWN:0002",
  "gene_symbol": "VWA5B1",
  "gene": "UniProtKB:Q5TIE3"
}